{
  "gene_name": "E3 ubiquitin-protein ligase TRIM58",
  "gene": "UniProtKB:Q8NG06",
  "gene_symbol": "TRIM58",
  "term_id": "GO:0061630",
  "term_label": "ubiquitin protein ligase activity"
}